{
  "gene_name": "Zygote arrest protein 1",
  "term_label": "negative regulation of translation",
  "term_id": "GO:0017148",
  "gene_symbol": "ZAR1",
  "gene": "UniProtKB:Q86SH2"
}